{
  "term_label": "Unknown biological process",
  "gene": "UniProtKB:P35325",
  "gene_name": "Small proline-rich protein 2B",
  "term_id": "UNKNOWN:0002",
  "gene_symbol": "SPRR2B"
}